{
  "term_label": "Unknown molecular function",
  "gene_symbol": "SPACA6",
  "gene": "UniProtKB:W5XKT8",
  "gene_name": "Sperm acrosome membrane-associated protein 6",
  "term_id": "UNKNOWN:0001"
}